{
  "gene_name": "Phospholipid-transporting ATPase IK",
  "gene": "UniProtKB:O60423",
  "term_label": "phospholipid translocation",
  "gene_symbol": "ATP8B3",
  "term_id": "GO:0045332"
}